{
  "gene_name": "Dapper homolog 1",
  "gene": "UniProtKB:Q9NYF0",
  "term_label": "regulation of Wnt signaling pathway, planar cell polarity pathway",
  "gene_symbol": "DACT1",
  "term_id": "GO:2000095"
}